cellular response to prostaglandin F stimulus [GO:0071381] (BP) Relationships: is a type of response to prostaglandin F [GO:0034696]; is a type of cellular response to prostaglandin stimulus [GO:0071379] Sources: GOC:mah Definition: Any process that results in a change in state or activity of a cell (in terms of movement, secretion, enzyme production, gene expression, etc.) as a result of a prostagladin F stimulus.